{
  "gene_symbol": "DNAJA2",
  "term_label": "unfolded protein binding",
  "gene_name": "DnaJ homolog subfamily A member 2",
  "gene": "UniProtKB:O60884",
  "term_id": "GO:0051082"
}